{
  "gene": "UniProtKB:Q9Y2R9",
  "gene_name": "Small ribosomal subunit protein uS7m",
  "term_label": "translation",
  "gene_symbol": "MRPS7",
  "term_id": "GO:0006412"
}